{
  "term_label": "DNA replication",
  "gene_name": "Replication protein A 70 kDa DNA-binding subunit",
  "gene": "UniProtKB:P27694",
  "gene_symbol": "RPA1",
  "term_id": "GO:0006260"
}